{
  "gene_symbol": "ADD1",
  "gene": "UniProtKB:P35611",
  "term_id": "GO:0005886",
  "term_label": "plasma membrane",
  "gene_name": "Alpha-adducin"
}